{
  "gene_symbol": "PPP2R2C",
  "gene": "UniProtKB:Q9Y2T4",
  "gene_name": "Serine_threonine-protein phosphatase 2A 55 kDa regulatory subunit B gamma isoform",
  "term_label": "protein phosphatase type 2A complex",
  "term_id": "GO:0000159"
}